THO complex part of transcription export complex [GO:0000445] (cellular component) Definition: The THO complex when it is part of the TREX (TRanscription EXport) complex that is involved in coupling transcription to export of mRNAs to the cytoplasm. In S. cerevisiae, it is composed of four subunits: Hpr1, Tho2, Thp1, and Mft1, while the human complex is composed of 7 subunits. References: PMID:11060033, PMID:11979277, PMID:16983072 Sources: GOC:krc Also known as: THO complex part of TREX complex Relationships: is a type of THO complex [GO:0000347]; is part of GO:0000346